stomach pylorus smooth muscle contraction [GO:0120064] (biological process) Definition: A process in which force is generated within gastric smooth muscle tissue, resulting in a change in muscle geometry. This process occurs in the most distal part of the stomach. Relationships: is a type of distal stomach smooth muscle contraction [GO:0014828] References: PMID:15890336 Sources: GOC:sl Subtypes: pyloric antrum smooth muscle contraction [GO:0120065], GO:0120066, pyloric sphincter smooth muscle contraction [GO:0120067]